{
  "term_id": "GO:0046330",
  "term_label": "positive regulation of JNK cascade",
  "gene_symbol": "TAOK2",
  "gene": "UniProtKB:Q9UL54",
  "gene_name": "Serine_threonine-protein kinase TAO2"
}